{
  "term_id": "GO:0047496",
  "gene_symbol": "HAP1",
  "term_label": "vesicle transport along microtubule",
  "gene_name": "Huntingtin-associated protein 1",
  "gene": "UniProtKB:P54257"
}